regulation of plasma cell differentiation [GO:1900098] (biological process) Definition: Any process that modulates the frequency, rate or extent of plasma cell differentiation. Sources: GOC:TermGenie Also known as: regulation of plasma cell development Relationships: is a type of regulation of immune effector process [GO:0002697]; is a type of regulation of B cell differentiation [GO:0045577]; is a type of regulation of immune response [GO:0050776]; regulates GO:0002317 Subtypes: GO:1900099, positive regulation of plasma cell differentiation [GO:1900100]